{
  "gene_symbol": "VIPAS39",
  "term_label": "vacuolar transport",
  "gene_name": "Spermatogenesis-defective protein 39 homolog",
  "term_id": "GO:0007034",
  "gene": "UniProtKB:Q9H9C1"
}